{
  "gene": "UniProtKB:P17024",
  "gene_name": "Zinc finger protein 20",
  "term_id": "GO:0005634",
  "term_label": "nucleus",
  "gene_symbol": "ZNF20"
}